oligosaccharyl transferase activity [GO:0004576] (molecular function) Definition: Catalysis of the transfer of a oligosaccharyl group to an acceptor molecule, typically another carbohydrate or a lipid. Sources: GOC:ai Also known as: oligosaccharide transferase activity Relationships: is a type of hexosyltransferase activity [GO:0016758] Subtypes: dolichyl-diphosphooligosaccharide-protein glycotransferase activity [GO:0004579]